{
  "gene_name": "Retinoic acid receptor RXR-beta",
  "term_label": "retinoic acid receptor signaling pathway",
  "gene_symbol": "RXRB",
  "gene": "UniProtKB:P28702",
  "term_id": "GO:0048384"
}